{
  "gene": "UniProtKB:Q9UFH2",
  "term_label": "dynein intermediate chain binding",
  "gene_name": "Dynein axonemal heavy chain 17",
  "term_id": "GO:0045505",
  "gene_symbol": "DNAH17"
}